{
  "term_id": "GO:0007216",
  "term_label": "G protein-coupled glutamate receptor signaling pathway",
  "gene": "UniProtKB:Q13255",
  "gene_symbol": "GRM1",
  "gene_name": "Metabotropic glutamate receptor 1"
}